{
  "term_id": "UNKNOWN:0002",
  "term_label": "Unknown biological process",
  "gene": "UniProtKB:Q14703",
  "gene_symbol": "MBTPS1",
  "gene_name": "Membrane-bound transcription factor site-1 protease"
}